{
  "gene": "UniProtKB:Q6UVM3",
  "term_label": "plasma membrane",
  "term_id": "GO:0005886",
  "gene_symbol": "KCNT2",
  "gene_name": "Potassium channel subfamily T member 2"
}